water-soluble vitamin catabolic process [GO:0042365] (BP) Definition: The chemical reactions and pathways resulting in the breakdown of any of a diverse group of vitamins that are soluble in water. References: PMID:24365359 Sources: GOC:jl Also known as: water-soluble vitamin breakdown, water-soluble vitamin catabolism, water-soluble vitamin degradation Relationships: is a type of vitamin catabolic process [GO:0009111] Subtypes: riboflavin catabolic process [GO:0009232], pantothenate catabolic process [GO:0015941], GO:0019854, cobalamin catabolic process [GO:0042366], GO:0042367, thiamine-containing compound catabolic process [GO:0042725], vitamin B6 catabolic process [GO:0042820], folic acid catabolic process [GO:0046657]